adenosine transport [GO:0032238] (biological process) Regulation: regulated by GO:0032249; RO_0002212 by negative regulation of adenosine transport [GO:0032250]; positively regulated by positive regulation of adenosine transport [GO:0032251] Relationships: is a type of nucleoside transport [GO:0015858] Definition: The directed movement of adenosine, adenine riboside, into, out of or within a cell, or between cells, by means of some agent such as a transporter or pore. Sources: GOC:mah